{
  "gene_name": "CKLF-like MARVEL transmembrane domain-containing protein 2",
  "gene": "UniProtKB:Q8TAZ6",
  "term_label": "membrane",
  "gene_symbol": "CMTM2",
  "term_id": "GO:0016020"
}